{
  "gene_symbol": "TDP1",
  "term_id": "GO:0006281",
  "term_label": "DNA repair",
  "gene": "UniProtKB:Q9NUW8",
  "gene_name": "Tyrosyl-DNA phosphodiesterase 1"
}